L-arginine transmembrane transporter activity [GO:0061459] (molecular function) Relationships: is a type of basic amino acid transmembrane transporter activity [GO:0015174]; is a type of GO:0015179; is part of L-arginine transmembrane transport [GO:1903826] Sources: GOC:dph Subtypes: GO:0005289, GO:0097626, L-lysine:L-arginine antiporter activity [GO:0106439] Also known as: arginine permease activity, L-arginine transporter activity, arginine transmembrane transporter activity, ATP-dependent L-arginine transmembrane transporter activity, ATPase-coupled L-arginine transmembrane transporter activity, L-arginine-importing ATPase activity, arginine porter activity, arginine-importing ATPase activity, histidine/arginine/lysine/ornithine porter activity Definition: Enables the transfer of L-arginine from one side of a membrane to the other.